{
  "gene_symbol": "MAP3K13",
  "gene": "UniProtKB:O43283",
  "term_label": "stress-activated MAPK cascade",
  "term_id": "GO:0051403",
  "gene_name": "Mitogen-activated protein kinase kinase kinase 13"
}